{
  "gene_name": "Serine_threonine-protein phosphatase 2A 55 kDa regulatory subunit B delta isoform",
  "term_label": "Unknown biological process",
  "gene_symbol": "PPP2R2D",
  "gene": "UniProtKB:Q66LE6",
  "term_id": "UNKNOWN:0002"
}